{
  "gene_symbol": "PHB1",
  "term_label": "Unknown molecular function",
  "gene_name": "Prohibitin 1",
  "gene": "UniProtKB:P35232",
  "term_id": "UNKNOWN:0001"
}